{
  "term_label": "transmembrane transporter activity",
  "gene": "UniProtKB:Q6ZSM3",
  "gene_symbol": "SLC16A12",
  "term_id": "GO:0022857",
  "gene_name": "Monocarboxylate transporter 12"
}